{
  "gene_symbol": "POLK",
  "gene_name": "DNA polymerase kappa",
  "term_label": "nucleus",
  "gene": "UniProtKB:Q9UBT6",
  "term_id": "GO:0005634"
}